{
  "term_label": "Golgi-associated vesicle",
  "gene_name": "Microtubule-associated protein 6",
  "term_id": "GO:0005798",
  "gene_symbol": "MAP6",
  "gene": "UniProtKB:Q96JE9"
}